{
  "term_label": "Unknown molecular function",
  "gene": "UniProtKB:Q8NA66",
  "gene_name": "Cyclic nucleotide-binding domain-containing protein 1",
  "term_id": "UNKNOWN:0001",
  "gene_symbol": "CNBD1"
}